{
  "gene_symbol": "RAD1",
  "term_label": "DNA damage checkpoint signaling",
  "term_id": "GO:0000077",
  "gene_name": "Cell cycle checkpoint protein RAD1",
  "gene": "UniProtKB:O60671"
}